{
  "term_label": "Unknown molecular function",
  "gene_name": "Carboxymethylenebutenolidase homolog",
  "gene": "UniProtKB:Q96DG6",
  "term_id": "UNKNOWN:0001",
  "gene_symbol": "CMBL"
}